{
  "gene_symbol": "MACF1",
  "term_id": "GO:0042060",
  "term_label": "wound healing",
  "gene_name": "Microtubule-actin cross-linking factor 1, isoforms 1_2_3_4_5",
  "gene": "UniProtKB:Q9UPN3"
}